lysophospholipase activity [GO:0120558] (molecular function) Relationships: is a type of phospholipase activity [GO:0004620]; is a type of carboxylic ester hydrolase activity [GO:0052689] Subtypes: GO:0004622, phosphatidylethanolamine lysophospholipase activity [GO:0120559], phosphatidylserine lysophospholipase activity [GO:0120560], phosphatidylinositol lysophospholipase activity [GO:0120561] Definition: Catalysis of the hydrolysis of a lysophospholipid (a phospholipid missing one fatty acid), removing the remaining acyl chain to yield a glycerophospho-compound and a free fatty acid. Sources: GOC:curators